{
  "term_label": "nucleus",
  "gene_name": "Putative fatty acid-binding protein 5-like protein 3",
  "gene": "UniProtKB:A8MUU1",
  "gene_symbol": "FABP5P3",
  "term_id": "GO:0005634"
}